{
  "gene": "UniProtKB:Q5T1V6",
  "gene_name": "Probable ATP-dependent RNA helicase DDX59",
  "term_label": "mRNA binding",
  "term_id": "GO:0003729",
  "gene_symbol": "DDX59"
}